regulation of translation in response to osmotic stress [GO:0043557] (biological process) Subtypes: negative regulation of translation in response to osmotic stress [GO:0032061], GO:0032062, regulation of translational initiation in response to osmotic stress [GO:0043561] Sources: GOC:jl Relationships: is a type of GO:0043555; is part of GO:0071470 Definition: Any process that modulates the frequency, rate or extent of the frequency, rate or extent of translation as a result of a stimulus indicating an increase or decrease in the concentration of solutes outside the organism or cell.